{
  "term_label": "proteasome regulatory particle",
  "term_id": "GO:0005838",
  "gene": "UniProtKB:Q15008",
  "gene_name": "26S proteasome non-ATPase regulatory subunit 6",
  "gene_symbol": "PSMD6"
}